{
  "term_label": "Unknown cellular component",
  "gene": "UniProtKB:Q96KR1",
  "term_id": "UNKNOWN:0003",
  "gene_name": "Zinc finger RNA-binding protein",
  "gene_symbol": "ZFR"
}